{
  "term_id": "UNKNOWN:0002",
  "gene_symbol": "PNMA3",
  "gene_name": "Paraneoplastic antigen Ma3",
  "gene": "UniProtKB:Q9UL41",
  "term_label": "Unknown biological process"
}